'de novo' AMP biosynthetic process [GO:0044208] (biological process) References: PMID:10888601 Sources: GOC:ecd Relationships: is a type of AMP biosynthetic process [GO:0006167] Definition: The chemical reactions and pathways resulting in the formation of adenosine monophosphate (AMP) from inosine 5'-monophosphate (IMP).